negative regulation of protein exit from endoplasmic reticulum [GO:0070862] (biological process) Definition: Any process that stops, prevents, or reduces the frequency, rate or extent of the directed movement of proteins from the endoplasmic reticulum. Sources: GOC:mah Also known as: down regulation of protein exit from endoplasmic reticulum, down-regulation of protein exit from endoplasmic reticulum, downregulation of protein exit from endoplasmic reticulum, negative regulation of protein exit from ER, negative regulation of protein export from ER, negative regulation of protein export from endoplasmic reticulum, inhibition of protein exit from endoplasmic reticulum Relationships: is a type of regulation of protein exit from endoplasmic reticulum [GO:0070861]; is a type of negative regulation of intracellular protein transport [GO:0090317]; negatively regulates GO:0032527 Subtypes: negative regulation of retrograde protein transport, ER to cytosol [GO:1904153]